{
  "gene": "UniProtKB:Q5VWK0",
  "term_label": "Unknown molecular function",
  "term_id": "UNKNOWN:0001",
  "gene_name": "Neuroblastoma breakpoint family member 6",
  "gene_symbol": "NBPF6"
}